acidocalcisome organization [GO:0106117] (biological process) References: PMID:25964650, PMID:26523947 Sources: GO:0020022 Relationships: is_a GO:0006996 Definition: A process that is carried out at the cellular level which results in the assembly, arrangement of constituent parts, or disassembly of an acidocalcisome. An acidocalcisome is an electron-dense acidic membrane-bounded organelle which contains a matrix of pyrophosphate and polyphosphates with bound calcium and other cations. Also known as: acidocalcisome biogenesis, acidocalcisome organisation, acidocalcisome organization and biogenesis, metachromatic granule organization, volutin granule organization, polyphosphate vacuole organization